{
  "gene": "UniProtKB:Q8WV28",
  "term_label": "cytoplasm",
  "gene_name": "B-cell linker protein",
  "gene_symbol": "BLNK",
  "term_id": "GO:0005737"
}